{
  "gene": "UniProtKB:P02654",
  "term_label": "very-low-density lipoprotein particle clearance",
  "gene_name": "Apolipoprotein C-I",
  "term_id": "GO:0034447",
  "gene_symbol": "APOC1"
}